{
  "gene_name": "Zinc finger protein 280D",
  "gene_symbol": "ZNF280D",
  "term_label": "regulation of DNA-templated transcription",
  "term_id": "GO:0006355",
  "gene": "UniProtKB:Q6N043"
}